positive regulation of telomerase RNA localization to Cajal body [GO:1904874] (biological process) Also known as: up regulation of telomerase RNA localization to Cajal body, up-regulation of telomerase RNA localization to Cajal body, upregulation of telomerase RNA localization to Cajal body, activation of telomerase RNA localization to Cajal body Definition: Any process that activates or increases the frequency, rate or extent of telomerase RNA localization to Cajal body. References: PMID:25467444 Sources: GOC:BHF, GOC:BHF_telomere, GOC:TermGenie, GOC:nc, GO_REF:0000058 Relationships: is a type of GO:0048518; is a type of regulation of telomerase RNA localization to Cajal body [GO:1904872]; positively regulates telomerase RNA localization to Cajal body [GO:0090671]